nuclear mRNA surveillance [GO:0071028] (biological process) Also known as: nuclear aberrant mRNA catabolic process, nuclear mRNA quality control, nuclear retention of pre-mRNA at the site of transcription, nuclear retention of pre-mRNA with aberrant 3'-ends at the site of transcription, nuclear retention of unspliced pre-mRNA at the site of transcription Subtypes: nuclear mRNA surveillance of meiosis-specific transcripts [GO:0033621], GO:0071030, nuclear mRNA surveillance of mRNA 3'-end processing [GO:0071031], nuclear mRNA surveillance of mRNP export [GO:0071032] Definition: A process that identifies and degrades defective or aberrant mRNAs within the nucleus. References: PMID:11586364, PMID:12417728, PMID:14718167, PMID:18644474 Sources: GOC:dgf, GOC:krc Relationships: is a type of GO:0000956; is a type of nuclear RNA surveillance [GO:0071027]